{
  "gene_name": "TATA-box-binding protein",
  "gene_symbol": "TBP",
  "gene": "UniProtKB:P20226",
  "term_label": "RNA polymerase II general transcription initiation factor activity",
  "term_id": "GO:0016251"
}